{
  "gene_symbol": "PMS2",
  "gene_name": "Mismatch repair endonuclease PMS2",
  "term_label": "MutLalpha complex",
  "gene": "UniProtKB:P54278",
  "term_id": "GO:0032389"
}